venom-mediated plasminogen activation [GO:0044544] (biological process) Also known as: envenomation resulting in plasminogen activation in another organism, envenomation resulting in plasminogen activation in other organism Definition: A process in which an organism initiates, promotes, or enhances the activation of plasminogen into plasmin in another organism via the action of a venom. This process includes cleavage at an internal Arg-Val site to form an N-terminal A-chain and C-terminal B-chain held together by a disulfide bond, and can include further proteolytic cleavage events to remove the preactivation peptide. Sources: GOC:fj, GOC:jl Relationships: is a type of venom-mediated fibrinolysis [GO:0044484]